{
  "gene_name": "Adenomatous polyposis coli protein",
  "term_label": "cell fate specification",
  "gene": "UniProtKB:P25054",
  "gene_symbol": "APC",
  "term_id": "GO:0001708"
}